{
  "term_id": "GO:0004674",
  "gene_name": "Serine_threonine-protein kinase 38-like",
  "gene_symbol": "STK38L",
  "term_label": "protein serine/threonine kinase activity",
  "gene": "UniProtKB:Q9Y2H1"
}